{
  "term_label": "nucleus",
  "gene_symbol": "CHCHD10",
  "gene": "UniProtKB:Q8WYQ3",
  "term_id": "GO:0005634",
  "gene_name": "Coiled-coil-helix-coiled-coil-helix domain-containing protein 10, mitochondrial"
}